{
  "term_label": "transport vesicle",
  "gene_name": "Biogenesis of lysosome-related organelles complex 1 subunit 6",
  "gene_symbol": "BLOC1S6",
  "term_id": "GO:0030133",
  "gene": "UniProtKB:Q9UL45"
}